{
  "gene_symbol": "KRTAP10-7",
  "gene": "UniProtKB:P60409",
  "term_id": "UNKNOWN:0002",
  "gene_name": "Keratin-associated protein 10-7",
  "term_label": "Unknown biological process"
}